{
  "gene": "UniProtKB:Q86XA9",
  "gene_symbol": "HEATR5A",
  "term_id": "GO:0006897",
  "term_label": "endocytosis",
  "gene_name": "HEAT repeat-containing protein 5A"
}